{
  "term_label": "fatty acid beta-oxidation using acyl-CoA dehydrogenase",
  "gene": "UniProtKB:P11310",
  "gene_name": "Medium-chain specific acyl-CoA dehydrogenase, mitochondrial",
  "term_id": "GO:0033539",
  "gene_symbol": "ACADM"
}